histone H3R2 methyltransferase activity [GO:0070611] (molecular function) Relationships: is a type of protein-arginine N-methyltransferase activity [GO:0016274]; is a type of GO:0140938 References: PMID:17898714 Also known as: histone H3R2 arginine methyltransferase activity, histone methylase activity (H3-R2 specific), histone methyltransferase activity (H3-R2 specific), histone-H3R2 methyltransferase activity, histone-arginine N-methyltransferase activity (H3-R2 specific) Definition: Catalysis of the reaction: S-adenosyl-L-methionine + (histone H3)-arginine (position 2) = S-adenosyl-L-homocysteine + (histone H3)-N-methyl-arginine (position 2). This reaction is the addition of a methyl group to the arginine residue at position 2 of histone H3. Note: Comment: Note that the residue position corresponds to the canonical human H3 histone (UniProtKB:P84243); this residue is conserved across all eukaryotes. Residue 1 is the first residue following removal of the initiating Methionine (Met). Note that each histone is encoded by multiple genes, and sequences may vary across different genes within an organism.